{
  "gene_symbol": "OR8K3",
  "term_id": "UNKNOWN:0003",
  "term_label": "Unknown cellular component",
  "gene_name": "Olfactory receptor 8K3",
  "gene": "UniProtKB:Q8NH51"
}